{
  "gene": "UniProtKB:Q7Z624",
  "term_label": "Unknown cellular component",
  "gene_name": "Calmodulin-lysine N-methyltransferase",
  "gene_symbol": "CAMKMT",
  "term_id": "UNKNOWN:0003"
}